{
  "term_id": "GO:0003712",
  "term_label": "transcription coregulator activity",
  "gene_symbol": "PHF2",
  "gene_name": "Lysine-specific demethylase PHF2",
  "gene": "UniProtKB:O75151"
}